eosinophil mediated immunity [GO:0002447] (BP) Definition: Any process involved in the carrying out of an immune response by an eosinophil. Sources: GOC:add, GO_REF:0000022, ISBN:0781735149 Relationships: is a type of GO:0002444